positive regulation of reactive oxygen species biosynthetic process [GO:1903428] (biological process) Subtypes: GO:0010729 Relationships: is_a GO:0009891; is a type of GO:1903426; is a type of positive regulation of reactive oxygen species metabolic process [GO:2000379]; positively regulates reactive oxygen species biosynthetic process [GO:1903409] References: PMID:24252804 Sources: GOC:PARL, GOC:TermGenie, GOC:bf, GO_REF:0000058 Definition: Any process that activates or increases the frequency, rate or extent of reactive oxygen species biosynthetic process. Also known as: positive regulation of reactive oxygen species anabolism, positive regulation of reactive oxygen species biosynthesis, positive regulation of reactive oxygen species formation, positive regulation of reactive oxygen species synthesis, up regulation of reactive oxygen species anabolism, up regulation of reactive oxygen species biosynthesis, up regulation of reactive oxygen species biosynthetic process, up regulation of reactive oxygen species formation, up regulation of reactive oxygen species synthesis, up-regulation of reactive oxygen species anabolism, up-regulation of reactive oxygen species biosynthesis, up-regulation of reactive oxygen species biosynthetic process, up-regulation of reactive oxygen species formation, up-regulation of reactive oxygen species synthesis, upregulation of reactive oxygen species anabolism, upregulation of reactive oxygen species biosynthesis, upregulation of reactive oxygen species biosynthetic process, upregulation of reactive oxygen species formation, upregulation of reactive oxygen species synthesis, activation of reactive oxygen species anabolism, activation of reactive oxygen species biosynthesis, activation of reactive oxygen species biosynthetic process, activation of reactive oxygen species formation, activation of reactive oxygen species synthesis, activation of ROS formation, activation of ROS generation, activation of reactive oxygen species generation, positive regulation of ROS formation, positive regulation of ROS generation, positive regulation of reactive oxygen species generation, up regulation of ROS formation, up regulation of ROS generation, up regulation of reactive oxygen species generation, up-regulation of ROS formation, up-regulation of ROS generation, up-regulation of reactive oxygen species generation, upregulation of ROS formation, upregulation of ROS generation, upregulation of reactive oxygen species generation